{
  "gene_symbol": "C4orf45",
  "gene_name": "Uncharacterized protein C4orf45",
  "term_label": "Unknown biological process",
  "gene": "UniProtKB:Q96LM5",
  "term_id": "UNKNOWN:0002"
}